{
  "gene": "UniProtKB:A6NNC1",
  "term_id": "UNKNOWN:0001",
  "gene_name": "Putative POM121-like protein 1-like",
  "term_label": "Unknown molecular function",
  "gene_symbol": "A6NNC1"
}